{
  "term_label": "brain development",
  "gene": "UniProtKB:Q6ISB3",
  "gene_name": "Grainyhead-like protein 2 homolog",
  "gene_symbol": "GRHL2",
  "term_id": "GO:0007420"
}